succinate-CoA ligase (GDP-forming) activity [GO:0004776] (molecular function) Definition: Catalysis of the reaction: GTP + succinate + CoA = GDP + succinyl-CoA + phosphate. Also known as: succinyl coenzyme A synthetase, succinate:CoA ligase (GDP-forming) activity, succinyl CoA synthetase activity, succinyl coenzyme A synthetase (GDP-forming) activity, succinyl coenzyme A synthetase (guanosine diphosphate-forming) activity, succinyl-CoA synthetase (GDP-forming) activity Sources: RHEA:22120 Relationships: is a type of succinate-CoA ligase activity [GO:0004774]